{
  "gene_symbol": "ADORA2A",
  "term_label": "adenylate cyclase-activating G protein-coupled receptor signaling pathway",
  "gene_name": "Adenosine receptor A2a",
  "gene": "UniProtKB:P29274",
  "term_id": "GO:0007189"
}